{
  "term_label": "positive regulation of type I interferon production",
  "gene": "UniProtKB:Q86WV6",
  "gene_name": "Stimulator of interferon genes protein",
  "gene_symbol": "STING1",
  "term_id": "GO:0032481"
}